{
  "gene_name": "Mitogen-activated protein kinase kinase kinase 3",
  "term_label": "protein serine/threonine kinase activity",
  "term_id": "GO:0004674",
  "gene": "UniProtKB:Q99759",
  "gene_symbol": "MAP3K3"
}